{
  "gene_name": "Ubiquitin carboxyl-terminal hydrolase MINDY-2",
  "term_label": "K48-linked deubiquitinase activity",
  "term_id": "GO:1990380",
  "gene": "UniProtKB:Q8NBR6",
  "gene_symbol": "MINDY2"
}